{
  "term_label": "Unknown cellular component",
  "gene_name": "Aquaporin-1",
  "gene": "UniProtKB:P29972",
  "term_id": "UNKNOWN:0003",
  "gene_symbol": "AQP1"
}